{
  "term_label": "cell migration",
  "gene_symbol": "ITGB1",
  "gene_name": "Integrin beta-1",
  "term_id": "GO:0016477",
  "gene": "UniProtKB:P05556"
}